{
  "gene_name": "Histone acetyltransferase KAT7",
  "term_id": "GO:0006357",
  "gene_symbol": "KAT7",
  "gene": "UniProtKB:O95251",
  "term_label": "regulation of transcription by RNA polymerase II"
}